{
  "gene": "UniProtKB:Q86WN2",
  "gene_symbol": "IFNE",
  "term_id": "GO:0006959",
  "term_label": "humoral immune response",
  "gene_name": "Interferon epsilon"
}